{
  "gene_name": "Leucine-rich repeat and fibronectin type-III domain-containing protein 5",
  "term_label": "regulation of presynapse assembly",
  "gene_symbol": "LRFN5",
  "term_id": "GO:1905606",
  "gene": "UniProtKB:Q96NI6"
}